{
  "term_id": "GO:0030522",
  "gene_name": "Vitamin D3 receptor",
  "gene": "UniProtKB:P11473",
  "term_label": "intracellular receptor signaling pathway",
  "gene_symbol": "VDR"
}